{
  "term_id": "GO:0000045",
  "gene_name": "Ras-related protein Rab-23",
  "term_label": "autophagosome assembly",
  "gene": "UniProtKB:Q9ULC3",
  "gene_symbol": "RAB23"
}